{
  "term_id": "GO:0004176",
  "gene_name": "ATP-dependent Clp protease proteolytic subunit, mitochondrial",
  "gene": "UniProtKB:Q16740",
  "term_label": "ATP-dependent peptidase activity",
  "gene_symbol": "CLPP"
}